{
  "term_label": "cytoplasm",
  "gene_name": "RAF proto-oncogene serine_threonine-protein kinase",
  "term_id": "GO:0005737",
  "gene": "UniProtKB:P04049",
  "gene_symbol": "RAF1"
}